{
  "term_label": "olfactory receptor activity",
  "term_id": "GO:0004984",
  "gene_name": "Olfactory receptor 4F15",
  "gene": "UniProtKB:Q8NGB8",
  "gene_symbol": "OR4F15"
}